{
  "gene_name": "Mpv17-like protein",
  "term_label": "Unknown molecular function",
  "gene": "UniProtKB:Q2QL34",
  "term_id": "UNKNOWN:0001",
  "gene_symbol": "MPV17L"
}